{
  "term_id": "GO:0004222",
  "gene_name": "Disintegrin and metalloproteinase domain-containing protein 22",
  "term_label": "metalloendopeptidase activity",
  "gene_symbol": "ADAM22",
  "gene": "UniProtKB:Q9P0K1"
}